{
  "gene_symbol": "CMPK2",
  "gene": "UniProtKB:Q5EBM0",
  "term_id": "GO:0006227",
  "term_label": "dUDP biosynthetic process",
  "gene_name": "UMP-CMP kinase 2, mitochondrial"
}